{
  "gene_name": "E3 ubiquitin-protein ligase RBX1",
  "gene": "UniProtKB:P62877",
  "term_label": "cullin family protein binding",
  "gene_symbol": "RBX1",
  "term_id": "GO:0097602"
}